{
  "term_label": "sodium ion transmembrane transport",
  "term_id": "GO:0035725",
  "gene_symbol": "SCN1A",
  "gene_name": "Sodium channel protein type 1 subunit alpha",
  "gene": "UniProtKB:P35498"
}